response to dimethyl sulfoxide [GO:1904619] (biological process) Relationships: is a type of response to chemical [GO:0042221] References: PMID:12873812 Sources: GOC:TermGenie, GO_REF:0000071 Also known as: response to DMSO Subtypes: cellular response to dimethyl sulfoxide [GO:1904620] Definition: Any process that results in a change in state or activity of a cell or an organism (in terms of movement, secretion, enzyme production, gene expression, etc.) as a result of a dimethyl sulfoxide stimulus.